regulation of maintenance of mitotic sister chromatid cohesion, arms [GO:2000715] (biological process) Definition: Any process that modulates the frequency, rate or extent of maintenance of mitotic sister chromatid cohesion along the chromosome arms. Sources: GOC:mah Also known as: regulation of maintenance of mitotic sister chromatin cohesion along arms, regulation of maintenance of sister chromatin cohesion along arms at mitosis Relationships: is a type of regulation of maintenance of mitotic sister chromatid cohesion [GO:0034182]; regulates maintenance of mitotic sister chromatid cohesion, arms [GO:0071959] Subtypes: negative regulation of maintenance of mitotic sister chromatid cohesion, arms [GO:2000716], positive regulation of maintenance of mitotic sister chromatid cohesion, arms [GO:2000717]